{
  "term_id": "GO:0000981",
  "gene_name": "Zinc finger protein 467",
  "gene": "UniProtKB:Q7Z7K2",
  "gene_symbol": "ZNF467",
  "term_label": "DNA-binding transcription factor activity, RNA polymerase II-specific"
}